positive regulation of nuclear-transcribed mRNA catabolic process, nonsense-mediated decay [GO:2000624] (biological process) Definition: Any process that activates or increases the frequency, rate or extent of nuclear-transcribed mRNA catabolic process, nonsense-mediated decay. Also known as: positive regulation of mRNA breakdown, nonsense-mediated decay, positive regulation of mRNA catabolic process, nonsense-mediated, positive regulation of mRNA catabolism, nonsense-mediated, positive regulation of mRNA degradation, nonsense-mediated decay, positive regulation of nonsense-mediated mRNA decay, positive regulation of nuclear mRNA catabolic process, nonsense-mediated decay Relationships: is a type of positive regulation of mRNA catabolic process [GO:0061014]; is a type of regulation of nuclear-transcribed mRNA catabolic process, nonsense-mediated decay [GO:2000622]; positively regulates GO:0000184 Sources: GOC:obol